{
  "gene_name": "COMM domain-containing protein 1",
  "term_id": "GO:1902306",
  "term_label": "negative regulation of sodium ion transmembrane transport",
  "gene_symbol": "COMMD1",
  "gene": "UniProtKB:Q8N668"
}